{
  "term_id": "GO:0005634",
  "gene": "UniProtKB:Q96AQ6",
  "gene_symbol": "PBXIP1",
  "gene_name": "Pre-B-cell leukemia transcription factor-interacting protein 1",
  "term_label": "nucleus"
}